cysteine-type exopeptidase activity [GO:0070004] (molecular function) Sources: GOC:mah, https://www.ebi.ac.uk/merops/about/glossary.shtml#CATTYPE, https://www.ebi.ac.uk/merops/about/glossary.shtml#EXOPEPTIDASE Subtypes: cysteine-type carboxypeptidase activity [GO:0016807], cysteine-type aminopeptidase activity [GO:0070005] Definition: Catalysis of the hydrolysis of C- or N-terminal peptide bonds in a polypeptide chain by a mechanism in which the sulfhydryl group of a cysteine residue at the active center acts as a nucleophile. Relationships: is a type of cysteine-type peptidase activity [GO:0008234]; is a type of exopeptidase activity [GO:0008238]